{
  "gene_symbol": "TRIM41",
  "term_id": "GO:0045087",
  "term_label": "innate immune response",
  "gene": "UniProtKB:Q8WV44",
  "gene_name": "E3 ubiquitin-protein ligase TRIM41"
}